{
  "term_label": "extracellular space",
  "gene": "UniProtKB:P14384",
  "term_id": "GO:0005615",
  "gene_name": "Carboxypeptidase M",
  "gene_symbol": "CPM"
}